{
  "gene": "UniProtKB:P53708",
  "gene_name": "Integrin alpha-8",
  "term_label": "cell surface",
  "gene_symbol": "ITGA8",
  "term_id": "GO:0009986"
}